{
  "gene_symbol": "LIPI",
  "term_id": "GO:0004620",
  "gene_name": "Lipase member I",
  "term_label": "phospholipase activity",
  "gene": "UniProtKB:Q6XZB0"
}